{
  "gene_name": "phospholipase A2 inhibitor and Ly6_PLAUR domain-containing protein",
  "gene_symbol": "PINLYP",
  "term_label": "Unknown cellular component",
  "gene": "UniProtKB:A6NC86",
  "term_id": "UNKNOWN:0003"
}